{
  "gene_name": "Eotaxin",
  "term_label": "chemokine activity",
  "gene_symbol": "CCL11",
  "term_id": "GO:0008009",
  "gene": "UniProtKB:P51671"
}